T-helper 1 cell extravasation [GO:0035687] (biological process) Relationships: is a type of helper T cell extravasation [GO:0035684]; is a type of GO:0035697 Definition: The migration of a T-helper 1 cell from the blood vessels into the surrounding tissue. A T-helper 1 cell is a CD4-positive, alpha-beta T cell that has the phenotype T-bet-positive and produces interferon-gamma. Also known as: Th1 cell extravasation Sources: CL:0000545, GOC:BHF